DNA recombinase mediator complex assembly [GO:1903871] (biological process) Also known as: DNA recombinase mediator complex formation Regulation: regulated by regulation of DNA recombinase mediator complex assembly [GO:1903872]; negatively regulated by negative regulation of DNA recombinase mediator complex assembly [GO:1903873] Relationships: is a type of DNA repair complex assembly [GO:0090735] Definition: The aggregation, arrangement and bonding together of a set of components to form a DNA recombinase mediator complex. References: PMID:18347097 Sources: GOC:TermGenie, GOC:rb, GO_REF:0000079